{
  "gene_name": "C-C chemokine receptor type 1",
  "term_label": "immune response",
  "gene": "UniProtKB:P32246",
  "gene_symbol": "CCR1",
  "term_id": "GO:0006955"
}